{
  "gene": "UniProtKB:Q96A57",
  "term_id": "GO:0008021",
  "gene_name": "Transmembrane protein 230",
  "term_label": "synaptic vesicle",
  "gene_symbol": "TMEM230"
}